Cdc48p-Npl4p-Vms1p AAA ATPase complex [GO:0036266] (cellular component) Relationships: is a type of outer mitochondrial membrane protein complex [GO:0098799] References: PMID:21070972, PMID:21936843 Sources: GOC:rn Definition: A multiprotein ATPase complex involved in the release of polyubiquitinated proteins, including those damaged by oxidative stress, from the outer mitochondria membrane into the cytoplasm where they are presented to the proteasome for proteolysis, a process also referred to as mitochondria-associated degradation (MAD). In budding yeast, this complex includes Cdc48p, Npl4p and Vms1p. Also known as: Cdc48p-Npl4p-Vms1p complex, Vms1-Cdc48-Npl4 complex, Vms1p-Cdc48p-Npl4p complex